{
  "gene_symbol": "YY1",
  "term_id": "GO:0031519",
  "gene": "UniProtKB:P25490",
  "gene_name": "Transcriptional repressor protein YY1",
  "term_label": "PcG protein complex"
}